{
  "gene_name": "Carbonic anhydrase 1",
  "gene_symbol": "CA1",
  "gene": "UniProtKB:P00915",
  "term_label": "carbonate dehydratase activity",
  "term_id": "GO:0004089"
}